{
  "gene_name": "GTPase RhebL1",
  "term_id": "GO:0003924",
  "gene": "UniProtKB:Q8TAI7",
  "term_label": "GTPase activity",
  "gene_symbol": "RHEBL1"
}